{
  "term_label": "small GTPase-mediated signal transduction",
  "term_id": "GO:0007264",
  "gene_name": "Rho guanine nucleotide exchange factor TIAM1",
  "gene_symbol": "TIAM1",
  "gene": "UniProtKB:Q13009"
}